{
  "gene": "UniProtKB:Q9NP80",
  "gene_symbol": "PNPLA8",
  "term_id": "GO:0016020",
  "term_label": "membrane",
  "gene_name": "Calcium-independent phospholipase A2-gamma"
}